{
  "term_id": "GO:0035725",
  "term_label": "sodium ion transmembrane transport",
  "gene": "UniProtKB:Q9UI33",
  "gene_name": "Sodium channel protein type 11 subunit alpha",
  "gene_symbol": "SCN11A"
}